{
  "gene_name": "Splicing factor, suppressor of white-apricot homolog",
  "gene": "UniProtKB:Q12872",
  "gene_symbol": "SFSWAP",
  "term_label": "Unknown molecular function",
  "term_id": "UNKNOWN:0001"
}